{
  "term_id": "GO:0035519",
  "gene_name": "RING-type domain-containing protein",
  "gene_symbol": "LOC122513141",
  "term_label": "protein K29-linked ubiquitination",
  "gene": "UniProtKB:A0A2R8Y4M4"
}